{
  "term_label": "Unknown biological process",
  "term_id": "UNKNOWN:0002",
  "gene_symbol": "TMEM92",
  "gene_name": "Transmembrane protein 92",
  "gene": "UniProtKB:Q6UXU6"
}